{
  "gene": "UniProtKB:Q5RL73",
  "gene_symbol": "RBM48",
  "term_label": "nucleoplasm",
  "term_id": "GO:0005654",
  "gene_name": "RNA-binding protein 48"
}